{
  "term_label": "diadenosine hexaphosphate catabolic process",
  "term_id": "GO:1901909",
  "gene": "UniProtKB:Q9NZJ9",
  "gene_name": "Diphosphoinositol polyphosphate phosphohydrolase 2",
  "gene_symbol": "NUDT4"
}